{
  "gene": "UniProtKB:Q14508",
  "term_id": "GO:0045087",
  "gene_name": "WAP four-disulfide core domain protein 2",
  "gene_symbol": "WFDC2",
  "term_label": "innate immune response"
}